{
  "gene_symbol": "SUMO2",
  "term_id": "GO:0044389",
  "gene": "UniProtKB:P61956",
  "term_label": "ubiquitin-like protein ligase binding",
  "gene_name": "Small ubiquitin-related modifier 2"
}